{
  "term_id": "GO:0050727",
  "gene_name": "B-cell lymphoma 6 protein",
  "term_label": "regulation of inflammatory response",
  "gene": "UniProtKB:P41182",
  "gene_symbol": "BCL6"
}